{
  "gene": "UniProtKB:Q9NYW3",
  "term_id": "GO:0001580",
  "term_label": "detection of chemical stimulus involved in sensory perception of bitter taste",
  "gene_symbol": "TAS2R7",
  "gene_name": "Taste receptor type 2 member 7"
}